{
  "term_id": "GO:0005737",
  "gene_name": "Kelch-like protein 40",
  "gene_symbol": "KLHL40",
  "gene": "UniProtKB:Q2TBA0",
  "term_label": "cytoplasm"
}